carbapenem biosynthetic process [GO:1901769] (biological process) Also known as: carbapenem anabolism, carbapenem biosynthesis, carbapenem formation, carbapenem synthesis Relationships: is a type of beta-lactam antibiotic biosynthetic process [GO:0030654] References: PMID:9402024 Sources: GOC:TermGenie, GOC:yaf, UniPathway:UPA00182 Definition: The chemical reactions and pathways resulting in the formation of carbapenem.